{
  "gene_name": "Immunoglobulin heavy variable 3-64",
  "term_id": "UNKNOWN:0003",
  "gene_symbol": "IGHV3-64",
  "gene": "UniProtKB:A0A075B6Q5",
  "term_label": "Unknown cellular component"
}